{
  "gene_symbol": "RNFT1",
  "term_id": "GO:1904294",
  "gene": "UniProtKB:Q5M7Z0",
  "gene_name": "E3 ubiquitin-protein ligase RNFT1",
  "term_label": "positive regulation of ERAD pathway"
}